{
  "gene_symbol": "SYT2",
  "term_id": "GO:0005886",
  "term_label": "plasma membrane",
  "gene": "UniProtKB:Q8N9I0",
  "gene_name": "Synaptotagmin-2"
}